positive regulation of cell proliferation involved in outflow tract morphogenesis [GO:1901964] (biological process) Relationships: is a type of GO:1901963; is_a positive regulation of cell proliferation involved in heart morphogenesis [GO:2000138]; positively regulates cell proliferation involved in outflow tract morphogenesis [GO:0061325] References: PMID:21419760 Sources: GOC:TermGenie, GOC:dph, GOC:mtg_heart Also known as: up regulation of cell proliferation involved in outflow tract morphogenesis, up-regulation of cell proliferation involved in outflow tract morphogenesis, upregulation of cell proliferation involved in outflow tract morphogenesis, activation of cell proliferation involved in outflow tract morphogenesis Definition: Any process that activates or increases the frequency, rate or extent of cell proliferation involved in outflow tract morphogenesis.